baroreceptor detection of decreased arterial stretch [GO:0003024] (biological process) Relationships: is a type of baroreceptor detection of arterial stretch [GO:0001981]; is part of baroreceptor response to decreased systemic arterial blood pressure [GO:0001982] Definition: The series of events by which a decrease in diameter of an artery is detected and converted to a molecular signal. Sources: GOC:mtg_cardio